mitochondrial protein-transporting ATPase activity [GO:0008566] (MF) Relationships: is a type of GO:0015450; occurs in mitochondrion [GO:0005739] Also known as: ATPase-coupled mitochondrial protein transporter activity Definition: Enables the transfer of a solute or solutes from one side of a membrane to the other according to the reaction: ATP + H2O = ADP + phosphate; drives the transport of proteins into the mitochondrion via the mitochondrial inner membrane translocase complex. Note: See also the cellular component term 'mitochondrial inner membrane presequence translocase complex ; GO:0005744'. Sources: EC:7.4.2.3